{
  "gene_name": "Plexin-A1",
  "term_label": "neuron projection guidance",
  "gene": "UniProtKB:Q9UIW2",
  "term_id": "GO:0097485",
  "gene_symbol": "PLXNA1"
}